mannosylglycerate transmembrane transporter activity [GO:0051477] (molecular function) References: PMID:15034926 Sources: GOC:ai Definition: Enables the transfer of a mannosylglycerate from one side of a membrane to the other. Relationships: is a type of carbohydrate transmembrane transporter activity [GO:0015144]; is a type of GO:0046943; is a type of GO:1901505; BFO_0000050 phosphoenolpyruvate-dependent mannosylglycerate phosphotransferase system [GO:0051476]